6-aminohexanoate transaminase activity [GO:0018719] (molecular function) Sources: UM-BBD_reactionID:r0449 Relationships: is a type of transaminase activity [GO:0008483] Definition: Catalysis of the reaction: 6-aminohexanoate + alpha-ketoglutarate = glutamate + 6-oxohexanoate.